keratinocyte development [GO:0003334] (biological process) Definition: The process whose specific outcome is the progression of a keratinocyte over time, from its formation to the mature structure. Relationships: is_a epithelial cell development [GO:0002064]; is part of keratinocyte differentiation [GO:0030216] Sources: GOC:dph